{
  "term_id": "UNKNOWN:0002",
  "gene_name": "tRNA-dihydrouridine(20a_20b) synthase [NAD(P)+]-like",
  "gene_symbol": "DUS4L",
  "gene": "UniProtKB:O95620",
  "term_label": "Unknown biological process"
}